{
  "gene": "UniProtKB:Q8TCP9",
  "gene_symbol": "FAM200A",
  "gene_name": "Protein FAM200A",
  "term_label": "Unknown molecular function",
  "term_id": "UNKNOWN:0001"
}